{
  "term_label": "cytoplasmic exosome (RNase complex)",
  "term_id": "GO:0000177",
  "gene_symbol": "EXOSC3",
  "gene_name": "Exosome complex component RRP40",
  "gene": "UniProtKB:Q9NQT5"
}